peptide secretion [GO:0002790] (biological process) Subtypes: antimicrobial peptide secretion [GO:0002776], peptide hormone secretion [GO:0030072], GO:0061544, orexin secretion [GO:0061584], GO:0099539 Relationships: is a type of peptide transport [GO:0015833]; is a type of GO:0046903 Regulation: regulated by regulation of peptide secretion [GO:0002791]; negatively regulated by negative regulation of peptide secretion [GO:0002792]; positively regulated by GO:0002793 Sources: GOC:add Definition: The controlled release of a peptide from a cell or a tissue.